{
  "gene": "UniProtKB:Q8TCQ1",
  "term_id": "GO:0002495",
  "gene_name": "E3 ubiquitin-protein ligase MARCHF1",
  "gene_symbol": "MARCHF1",
  "term_label": "antigen processing and presentation of peptide antigen via MHC class II"
}